peptidoglycan muralytic activity [GO:0061783] (molecular function) References: PMID:22748813 Sources: GOC:dph, GOC:jh Definition: A catalytic activity that contributes to the degradation of peptidoglycan. Subtypes: lysozyme activity [GO:0003796], N-acetylmuramoyl-L-alanine amidase activity [GO:0008745], peptidoglycan lytic transglycosylase activity [GO:0008933], peptidoglycan N-acetylglucosaminidase activity [GO:0061784], peptidoglycan endopeptidase activity [GO:0061785] Relationships: is a type of catalytic activity [GO:0003824]